{
  "gene": "UniProtKB:O00175",
  "term_id": "GO:0008009",
  "gene_symbol": "CCL24",
  "gene_name": "C-C motif chemokine 24",
  "term_label": "chemokine activity"
}